dihydroorotate dehydrogenase (quinone) activity [GO:0106430] (molecular function) Definition: (S)-dihydroorotate + a quinone = orotate + a quinol. Sources: RHEA:30187 Relationships: is a type of dihydroorotate dehydrogenase activity [GO:0004152]; is a type of oxidoreductase activity, acting on the CH-CH group of donors, quinone or related compound as acceptor [GO:0016635]